{
  "gene_symbol": "DCSTAMP",
  "term_label": "endoplasmic reticulum membrane",
  "gene_name": "Dendritic cell-specific transmembrane protein",
  "gene": "UniProtKB:Q9H295",
  "term_id": "GO:0005789"
}